{
  "gene": "UniProtKB:P48167",
  "term_label": "chloride channel activity",
  "gene_symbol": "GLRB",
  "term_id": "GO:0005254",
  "gene_name": "Glycine receptor subunit beta"
}